{
  "term_id": "GO:0007259",
  "gene_symbol": "STAT4",
  "term_label": "cell surface receptor signaling pathway via JAK-STAT",
  "gene_name": "Signal transducer and activator of transcription 4",
  "gene": "UniProtKB:Q14765"
}